detection of hypoxic conditions in blood by chemoreceptor signaling [GO:0002007] (biological process) Sources: GOC:dph Subtypes: detection of hypoxic conditions in blood by carotid body chemoreceptor signaling [GO:0003029], detection of hypoxic conditions in blood by aortic body chemoreceptor signaling [GO:0003033] Definition: The process in which information about a lack of oxygen are received and are converted to a molecular signal by chemoreceptors in the carotid bodies and the aortic bodies. Also known as: detection of hypoxic conditions in blood by chemoreceptor signalling Relationships: is a type of detection of chemical stimulus [GO:0009593]; is part of regulation of systemic arterial blood pressure by chemoreceptor signaling [GO:0001979]; BFO_0000050 cellular response to chemical stimulus [GO:0070887]; has part detection of pH by chemoreceptor signaling [GO:0003022]